lysosomal matrix [GO:1990836] (cellular component) Definition: A matrix composed of supramolecular assemblies of lysosomal enzymes and lipids which forms at a pH of 5.0 within the lysosome. References: PMID:9395337 Relationships: is a type of cellular anatomical structure [GO:0110165]; is part of GO:0043202